{
  "gene": "UniProtKB:Q96C55",
  "gene_name": "Zinc finger protein 524",
  "term_id": "UNKNOWN:0003",
  "gene_symbol": "ZNF524",
  "term_label": "Unknown cellular component"
}